{
  "term_id": "GO:0005886",
  "gene_name": "Tyrosine-protein kinase Blk",
  "gene": "UniProtKB:P51451",
  "gene_symbol": "BLK",
  "term_label": "plasma membrane"
}